{
  "term_label": "cytosol",
  "gene_name": "Cytosolic phospholipase A2 zeta",
  "gene": "UniProtKB:Q68DD2",
  "gene_symbol": "PLA2G4F",
  "term_id": "GO:0005829"
}